renal water transport [GO:0003097] (biological process) Regulation: regulated by regulation of renal water transport [GO:2001151]; negatively regulated by GO:2001152; positively regulated by positive regulation of renal water transport [GO:2001153] Relationships: is a type of renal system process [GO:0003014]; is a type of water transport [GO:0006833]; is part of renal water homeostasis [GO:0003091] Sources: GOC:mtg_cardio Subtypes: GO:0070295 Definition: The directed movement of water (H2O) by the renal system.